negative regulation of cap-dependent translational initiation [GO:1903675] (BP) Sources: GOC:PARL, GOC:TermGenie, GOC:bf, GO_REF:0000058 Definition: Any process that stops, prevents or reduces the frequency, rate or extent of cap-dependent translational initiation. Relationships: is a type of regulation of cap-dependent translational initiation [GO:1903674]; is_a GO:1904689; negatively regulates cap-dependent translational initiation [GO:0002191] Also known as: down regulation of cap-dependent translational initiation, down-regulation of cap-dependent translational initiation, downregulation of cap-dependent translational initiation, inhibition of cap-dependent translational initiation